deoxyinosine catabolic process [GO:0006149] (biological process) Also known as: deoxyinosine breakdown, deoxyinosine catabolism, deoxyinosine degradation Relationships: is a type of deoxyinosine metabolic process [GO:0046094]; is_a GO:0046124 Sources: GOC:go_curators Definition: The chemical reactions and pathways resulting in the breakdown of deoxyinosine, hypoxanthine deoxyriboside.